siRNA 3'-end processing [GO:1990432] (biological process) Relationships: is a type of regulatory ncRNA 3'-end processing [GO:0043628] References: PMID:24095277 Definition: The process of forming the mature 3' end of a siRNA molecule. Also known as: siRNA 3' end processing, small interfering RNA 3'-end processing